{
  "gene_symbol": "RASSF2",
  "gene_name": "Ras association domain-containing protein 2",
  "term_label": "nucleus",
  "term_id": "GO:0005634",
  "gene": "UniProtKB:P50749"
}